{
  "gene_name": "Beta-actin-like protein 2",
  "term_id": "GO:0030424",
  "term_label": "axon",
  "gene_symbol": "ACTBL2",
  "gene": "UniProtKB:Q562R1"
}